{
  "gene": "UniProtKB:Q9NXD2",
  "gene_name": "Myotubularin-related protein 10",
  "term_label": "Unknown biological process",
  "gene_symbol": "MTMR10",
  "term_id": "UNKNOWN:0002"
}